{
  "term_id": "UNKNOWN:0002",
  "gene_name": "Cortexin-3",
  "gene": "UniProtKB:Q4LDR2",
  "term_label": "Unknown biological process",
  "gene_symbol": "CTXN3"
}